regulation of ubiquitin-dependent endocytosis [GO:2000395] (biological process) Relationships: is a type of regulation of endocytosis [GO:0030100]; is a type of regulation of protein transport [GO:0051223]; regulates ubiquitin-dependent endocytosis [GO:0070086] Also known as: regulation of ubiquitin-mediated endocytosis Definition: Any process that modulates the frequency, rate or extent of ubiquitin-dependent endocytosis. Sources: GOC:mah Subtypes: negative regulation of ubiquitin-dependent endocytosis [GO:2000396], GO:2000397